acetoin metabolic process [GO:0045149] (biological process) Definition: The chemical reactions and pathways involving acetoin, 3-hydroxy-2-butanone, often as part of a fermentation pathway or for use as a carbon source. Sources: GOC:mlg Also known as: acetoin metabolism Relationships: is a type of ketone metabolic process [GO:0042180]; is a type of secondary alcohol metabolic process [GO:1902652] Subtypes: acetoin catabolic process [GO:0045150], acetoin biosynthetic process [GO:0045151]